{
  "term_label": "cytoplasm",
  "gene_symbol": "TRAF2",
  "gene": "UniProtKB:Q12933",
  "gene_name": "TNF receptor-associated factor 2",
  "term_id": "GO:0005737"
}